lateral mesoderm morphogenesis [GO:0048369] (biological process) Also known as: lateral plate mesoderm morphogenesis Sources: GOC:go_curators Definition: The process in which the anatomical structures of the lateral mesoderm are generated and organized. Relationships: is a type of mesoderm morphogenesis [GO:0048332]; is a type of mesenchyme morphogenesis [GO:0072132]; is part of lateral mesoderm development [GO:0048368]